{
  "gene_symbol": "SLCO1B3-SLCO1B7",
  "gene": "UniProtKB:F5H094",
  "term_label": "bile acid and bile salt transport",
  "term_id": "GO:0015721",
  "gene_name": "SLCO1B3-SLCO1B7 readthrough transcript protein"
}